{
  "term_id": "GO:0000922",
  "gene": "UniProtKB:Q6P4I2",
  "gene_symbol": "WDR73",
  "gene_name": "WD repeat-containing protein 73",
  "term_label": "spindle pole"
}